zinc export across plasma membrane [GO:0140882] (biological process) Relationships: is a type of GO:0071577; is a type of export across plasma membrane [GO:0140115] Definition: The directed movement of zinc ions from a cell, into the extracellular region. Also known as: zinc ion export from cell References: PMID:17355957